flavonoid binding [GO:0097243] (molecular function) References: PMID:20599706 Sources: GOC:sl Subtypes: flavonol binding [GO:0097244], flavanol binding [GO:0097245], epigallocatechin 3-gallate binding [GO:0097247], quercitrin binding [GO:2001227] Relationships: is a type of binding [GO:0005488] Definition: Binding to a flavonoid, a compound containing two or more aromatic rings, each bearing at least one aromatic hydroxyl and connected with a carbon bridge.